{
  "term_label": "beta-catenin destruction complex",
  "gene": "UniProtKB:Q9Y2T1",
  "gene_symbol": "AXIN2",
  "gene_name": "Axin-2",
  "term_id": "GO:0030877"
}